{
  "term_label": "vacuolar transport",
  "term_id": "GO:0007034",
  "gene_symbol": "ATP6V0D1",
  "gene": "UniProtKB:P61421",
  "gene_name": "V-type proton ATPase subunit d 1"
}